{
  "term_label": "mRNA binding",
  "gene": "UniProtKB:Q8NA57",
  "gene_name": "Uncharacterized protein C12orf50",
  "gene_symbol": "C12orf50",
  "term_id": "GO:0003729"
}